{
  "gene_symbol": "ALAD",
  "gene_name": "Delta-aminolevulinic acid dehydratase",
  "term_label": "porphobilinogen synthase activity",
  "term_id": "GO:0004655",
  "gene": "UniProtKB:P13716"
}